dTMP kinase activity [GO:0004798] (molecular function) Sources: RHEA:13517 Also known as: thymidylate kinase activity, ATP:dTMP phosphotransferase activity, TMPK activity, deoxythymidine 5'-monophosphate kinase activity, thymidine 5'-monophosphate kinase activity, thymidine monophosphate kinase activity, thymidylate monophosphate kinase activity, thymidylic acid kinase activity, thymidylic kinase activity Relationships: is a type of deoxynucleoside phosphate kinase activity, ATP as phosphate donor [GO:0047507] Definition: Catalysis of the reaction: dTMP + ATP = dTDP + ADP.